{
  "gene": "UniProtKB:Q9NRH1",
  "gene_name": "Protein YAE1 homolog",
  "gene_symbol": "YAE1",
  "term_label": "Unknown cellular component",
  "term_id": "UNKNOWN:0003"
}